positive regulation of lung alveolus development [GO:1904655] (biological process) Relationships: is a type of positive regulation of developmental process [GO:0051094]; is a type of positive regulation of multicellular organismal process [GO:0051240]; is_a GO:1904653; positively regulates GO:0048286 Also known as: positive regulation of alveolarization, positive regulation of alveologenesis, up regulation of alveolarization, up regulation of alveologenesis, up regulation of lung alveolus development, up-regulation of alveolarization, up-regulation of alveologenesis, up-regulation of lung alveolus development, upregulation of alveolarization, upregulation of alveologenesis, upregulation of lung alveolus development, activation of alveolarization, activation of alveologenesis, activation of lung alveolus development References: PMID:23962064 Sources: GOC:TermGenie, GO_REF:0000058 Definition: Any process that activates or increases the frequency, rate or extent of lung alveolus development.